acetate catabolic process [GO:0045733] (biological process) Definition: The chemical reactions and pathways resulting in the breakdown of acetate, the anion of acetic acid. Relationships: is a type of GO:0006083; is a type of monocarboxylic acid catabolic process [GO:0072329] Sources: GOC:go_curators Also known as: acetate breakdown, acetate catabolism, acetate degradation, homoacetate catabolic process Regulation: RO_0002211 by regulation of acetate catabolic process [GO:0045734]; negatively regulated by negative regulation of acetate catabolic process [GO:0045753]; positively regulated by GO:0045754